negative regulation of transcription by glucose [GO:0061986] (biological process) Definition: Any process involving glucose that decreases the frequency, rate or extent or transcription. References: PMID:11875061 Relationships: is_a regulation of transcription by glucose [GO:0046015] Subtypes: carbon catabolite repression of transcription by glucose [GO:0045014], negative regulation of transcription from RNA polymerase II promoter by glucose [GO:0061987]